{
  "term_id": "GO:0015937",
  "gene_symbol": "PANK2",
  "term_label": "coenzyme A biosynthetic process",
  "gene": "UniProtKB:Q9BZ23",
  "gene_name": "Pantothenate kinase 2, mitochondrial"
}